cuticular plate [GO:0032437] (cellular component) Definition: A dense network of actin filaments found beneath the apical cell surface of hair cells, and into which stereocilia are inserted. References: PMID:12485990, PMID:2592408, PMID:8071151 Relationships: is a type of cellular anatomical structure [GO:0110165]; is part of GO:0030864